{
  "gene_name": "Polyunsaturated fatty acid lipoxygenase ALOX15",
  "term_label": "cytosol",
  "term_id": "GO:0005829",
  "gene": "UniProtKB:P16050",
  "gene_symbol": "ALOX15"
}